{
  "term_label": "Unknown biological process",
  "term_id": "UNKNOWN:0002",
  "gene_symbol": "SGF29",
  "gene": "UniProtKB:Q96ES7",
  "gene_name": "SAGA-associated factor 29"
}